autolysosome membrane [GO:0120281] (cellular component) Definition: A lipid bilayer that surrounds an autolysosome, a single-membrane-bounded vesicle in which endogenous cellular material is degraded. Relationships: is a type of lysosomal membrane [GO:0005765]; is part of autolysosome [GO:0044754] References: PMID:17182262, PMID:24657946, PMID:26382870, PMID:32047650 Sources: GOC:krc, GOC:nhn